{
  "term_id": "GO:0019901",
  "gene_symbol": "SPRED2",
  "gene": "UniProtKB:Q7Z698",
  "gene_name": "Sprouty-related, EVH1 domain-containing protein 2",
  "term_label": "protein kinase binding"
}